shoot axis formation [GO:0010346] (biological process) Subtypes: secondary shoot formation [GO:0010223] Sources: GOC:tb Also known as: shoot formation Relationships: is a type of GO:1905393; is part of shoot system morphogenesis [GO:0010016] Definition: The process that gives rise to a shoot axis. This process pertains to the initial formation of a structure from unspecified parts.